{
  "gene": "UniProtKB:Q5JSJ4",
  "term_id": "GO:0030674",
  "term_label": "protein-macromolecule adaptor activity",
  "gene_symbol": "INTS6L",
  "gene_name": "Integrator complex subunit 6-like"
}